central nervous system myelin formation [GO:0032289] (biological process) Also known as: central nervous system myelin sheath formation, myelin formation in central nervous system Definition: The process in which the wraps of cell membrane that constitute myelin are laid down around an axon by an oligodendrocyte in the central nervous system. Relationships: is a type of myelin assembly [GO:0032288]; is part of central nervous system myelination [GO:0022010] Sources: GOC:dgh